{
  "gene_symbol": "ARPC1A",
  "gene": "UniProtKB:Q92747",
  "gene_name": "Actin-related protein 2_3 complex subunit 1A",
  "term_id": "GO:0051015",
  "term_label": "actin filament binding"
}